{
  "gene_name": "Protein PAXX",
  "gene": "UniProtKB:Q9BUH6",
  "term_label": "nucleus",
  "term_id": "GO:0005634",
  "gene_symbol": "PAXX"
}